mating-type locus imprinting [GO:0071515] (BP) Definition: A genomic imprinting process in which a stable single-strand DNA lesion triggers programmed gene conversion at the mating-type locus, thereby restricting mating-type interconversion to one of the two sister chromatids during DNA replication. References: PMID:14765111, PMID:18723894 Sources: GOC:mah Also known as: genetic imprinting at mating-type locus, genomic imprinting at mating-type locus, mating type determination, imprinting Relationships: is a type of GO:0022413; is part of GO:0007533